{
  "gene": "UniProtKB:Q9UKV8",
  "gene_name": "Protein argonaute-2",
  "term_id": "GO:0035198",
  "gene_symbol": "AGO2",
  "term_label": "miRNA binding"
}